{
  "gene_symbol": "EZR",
  "gene": "UniProtKB:P15311",
  "term_label": "positive regulation of protein localization to early endosome",
  "gene_name": "Ezrin",
  "term_id": "GO:1902966"
}